{
  "term_label": "Unknown biological process",
  "term_id": "UNKNOWN:0002",
  "gene_symbol": "CCDC196",
  "gene_name": "Putative coiled-coil domain-containing protein 196",
  "gene": "UniProtKB:A0A1B0GTZ2"
}